{
  "gene_symbol": "MRPL46",
  "gene_name": "Large ribosomal subunit protein mL46",
  "term_label": "structural constituent of ribosome",
  "gene": "UniProtKB:Q9H2W6",
  "term_id": "GO:0003735"
}